positive regulation of glucomannan catabolic process [GO:2000908] (biological process) Relationships: is_a regulation of glucomannan catabolic process [GO:2000898]; is a type of positive regulation of mannan catabolic process [GO:2000996]; positively regulates glucomannan catabolic process [GO:2000884] Sources: GOC:mengo_curators Also known as: positive regulation of glucomannan catabolism Definition: Any process that activates or increases the frequency, rate or extent of glucomannan catabolic process.